{
  "term_id": "GO:0007155",
  "gene": "UniProtKB:Q9Y5G2",
  "term_label": "cell adhesion",
  "gene_name": "Protocadherin gamma-B2",
  "gene_symbol": "PCDHGB2"
}